{
  "gene": "UniProtKB:O75569",
  "gene_symbol": "PRKRA",
  "term_id": "GO:0005737",
  "term_label": "cytoplasm",
  "gene_name": "Interferon-inducible double-stranded RNA-dependent protein kinase activator A"
}